{
  "gene_name": "Golgi phosphoprotein 3",
  "gene_symbol": "GOLPH3",
  "term_label": "Golgi vesicle budding",
  "gene": "UniProtKB:Q9H4A6",
  "term_id": "GO:0048194"
}